{
  "gene_symbol": "KIF5C",
  "term_id": "GO:0008017",
  "term_label": "microtubule binding",
  "gene_name": "Kinesin heavy chain isoform 5C",
  "gene": "UniProtKB:O60282"
}